{
  "term_id": "GO:0070102",
  "gene": "UniProtKB:P05231",
  "gene_symbol": "IL6",
  "gene_name": "Interleukin-6",
  "term_label": "interleukin-6-mediated signaling pathway"
}